{
  "gene_name": "Cell division cycle-associated protein 7",
  "gene": "UniProtKB:Q9BWT1",
  "gene_symbol": "CDCA7",
  "term_id": "GO:0005634",
  "term_label": "nucleus"
}